{
  "term_id": "UNKNOWN:0001",
  "gene": "UniProtKB:P0C7V4",
  "gene_symbol": "FAM90A15P",
  "term_label": "Unknown molecular function",
  "gene_name": "Putative protein FAM90A15P"
}